{
  "gene_symbol": "CBY2",
  "gene": "UniProtKB:Q8NA61",
  "term_id": "UNKNOWN:0002",
  "gene_name": "Protein chibby homolog 2",
  "term_label": "Unknown biological process"
}